MHC class I biosynthetic process [GO:0045341] (biological process) Relationships: is a type of macromolecule biosynthetic process [GO:0009059] Also known as: MHC class I anabolism, MHC class I biosynthesis, MHC class I formation, MHC class I synthesis, major histocompatibility complex class I biosynthesis, major histocompatibility complex class I biosynthetic process Sources: GOC:go_curators Regulation: regulated by regulation of MHC class I biosynthetic process [GO:0045343]; negatively regulated by negative regulation of MHC class I biosynthetic process [GO:0045344]; RO_0002213 by positive regulation of MHC class I biosynthetic process [GO:0045345] Definition: The chemical reactions and pathways resulting in the formation of major histocompatibility protein class I.